{
  "gene_name": "Tudor domain-containing protein 15",
  "term_id": "UNKNOWN:0003",
  "gene_symbol": "TDRD15",
  "gene": "UniProtKB:B5MCY1",
  "term_label": "Unknown cellular component"
}